{
  "gene": "UniProtKB:Q96DH6",
  "term_id": "GO:0003729",
  "term_label": "mRNA binding",
  "gene_symbol": "MSI2",
  "gene_name": "RNA-binding protein Musashi homolog 2"
}